{
  "gene": "UniProtKB:Q9NQ33",
  "term_label": "RNA polymerase II transcription regulatory region sequence-specific DNA binding",
  "term_id": "GO:0000977",
  "gene_name": "Achaete-scute homolog 3",
  "gene_symbol": "ASCL3"
}